mitotic anaphase A [GO:0000091] (biological process) Relationships: is a type of mitotic anaphase [GO:0000090] Definition: The cell cycle phase during which the kinetochore microtubules shorten as chromosomes move toward the spindle poles as part of mitosis. Note: Note that this term should not be used for direct annotation. If you are trying to make an annotation to x phase, it is likely that the correct annotation is 'regulation of x/y phase transition' or to a process which occurs during the reported phase (i.e mitotic DNA replication for mitotic S-phase). To capture the phase when a specific location or process is observed, the phase term can be used in an annotation extension (PMID:24885854) applied to a cellular component term (with the relation exists_during) or a biological process term (with the relation happens_during). Sources: GOC:mtg_cell_cycle